{
  "gene_name": "Pre-mRNA-processing factor 6",
  "term_label": "catalytic step 2 spliceosome",
  "gene": "UniProtKB:O94906",
  "term_id": "GO:0071013",
  "gene_symbol": "PRPF6"
}